{
  "gene_symbol": "LTC4S",
  "gene": "UniProtKB:Q16873",
  "gene_name": "Leukotriene C4 synthase",
  "term_id": "GO:0004602",
  "term_label": "glutathione peroxidase activity"
}